{
  "gene": "UniProtKB:P16615",
  "term_label": "regulation of cardiac muscle contraction by calcium ion signaling",
  "gene_symbol": "ATP2A2",
  "gene_name": "Sarcoplasmic_endoplasmic reticulum calcium ATPase 2",
  "term_id": "GO:0010882"
}